regulation of Toll receptor ligand protein activation cascade [GO:0160033] (biological process) References: PMID:23632253 Definition: Any process that modulates the frequency, rate or extent of the Toll receptor ligand protein activation cascade. Subtypes: positive regulation of Toll receptor ligand protein activation cascade [GO:0160034], GO:0160035 Relationships: is a type of regulation of protein activation cascade [GO:2000257]; RO_0002211 Toll receptor ligand protein activation cascade [GO:0160032]